{
  "gene_symbol": "HLA-DPB1",
  "term_id": "GO:0002503",
  "gene": "UniProtKB:P04440",
  "term_label": "peptide antigen assembly with MHC class II protein complex",
  "gene_name": "HLA class II histocompatibility antigen, DP beta 1 chain"
}